positive regulation of hair follicle maturation [GO:0048818] (biological process) Sources: GOC:devbiol Definition: Any process that activates or increases the frequency, rate or extent of hair follicle maturation. Subtypes: GO:0051795, positive regulation of timing of anagen [GO:0051885], positive regulation of timing of exogen [GO:0051888] Also known as: up regulation of hair follicle maturation, up-regulation of hair follicle maturation, upregulation of hair follicle maturation, activation of hair follicle maturation, stimulation of hair follicle maturation Relationships: is a type of regulation of hair follicle maturation [GO:0048819]; is a type of positive regulation of hair follicle development [GO:0051798]; positively regulates hair follicle maturation [GO:0048820]